pH-gated chloride channel activity [GO:0061797] (MF) Relationships: is_a chloride channel activity [GO:0005254]; is a type of GO:0099095; is a type of pH-gated monoatomic ion channel activity [GO:0160128] Definition: A gated channel activity that enables the transmembrane transfer of a chloride ion by a channel that opens in response to a change in pH. References: PMID:27358471 Sources: GOC:dph